{
  "gene_name": "Transmembrane 4 L6 family member 20",
  "term_label": "Unknown biological process",
  "term_id": "UNKNOWN:0002",
  "gene_symbol": "TM4SF20",
  "gene": "UniProtKB:Q53R12"
}